diacetyl reductase ((S)-acetoin forming) (NAD+) activity [GO:0052588] (molecular function) Definition: Catalysis of the reaction: (S)-acetoin + NAD+ = diacetyl + H+ + NADH. This reaction is catalyzed in the reverse direction. Sources: RHEA:27286 Also known as: (S)-acetoin dehydrogenase activity Relationships: is a type of acetoin dehydrogenase (NAD+) activity [GO:0019152]